{
  "gene_name": "LIM_homeobox protein Lhx2",
  "gene_symbol": "LHX2",
  "term_id": "GO:0000981",
  "gene": "UniProtKB:P50458",
  "term_label": "DNA-binding transcription factor activity, RNA polymerase II-specific"
}